regulation of thalamus size [GO:0090067] (biological process) Relationships: is_a regulation of anatomical structure size [GO:0090066] Definition: Any process that modulates the size of the thalamus. The thalamus is a part of the diencephalon that is composed of the dorsal thalamus and the ventral thalamus. Sources: GOC:dph, GOC:tb